{
  "term_label": "somatostatin receptor activity",
  "gene_symbol": "SSTR1",
  "gene_name": "Somatostatin receptor type 1",
  "gene": "UniProtKB:P30872",
  "term_id": "GO:0004994"
}